{
  "term_id": "GO:0000015",
  "gene_symbol": "ENO1",
  "gene_name": "Alpha-enolase",
  "term_label": "phosphopyruvate hydratase complex",
  "gene": "UniProtKB:P06733"
}